mechanosensory epithelium regeneration [GO:0070655] (biological process) Definition: The regrowth of lost or destroyed mechanosensory epithelia. References: PMID:19381250 Sources: GOC:dsf Subtypes: GO:0070657, inner ear sensory epithelium regeneration [GO:0070659] Relationships: is a type of sensory epithelium regeneration [GO:0070654]